{
  "gene": "UniProtKB:O60296",
  "term_id": "GO:0048311",
  "term_label": "mitochondrion distribution",
  "gene_name": "Trafficking kinesin-binding protein 2",
  "gene_symbol": "TRAK2"
}